{
  "gene_name": "Dopamine beta-hydroxylase",
  "term_id": "GO:0005507",
  "gene": "UniProtKB:P09172",
  "term_label": "copper ion binding",
  "gene_symbol": "DBH"
}